secondary cell septum biogenesis [GO:1990344] (biological process) Relationships: is a type of GO:0044085; is a type of GO:1902410; is part of GO:0140278 Definition: A cellular process that results in the biosynthesis of constituent macromolecules, assembly, and arrangement of constituent parts of a secondary cell septum following nuclear division. Regulation: regulated by regulation of secondary cell septum biogenesis [GO:1903395]; negatively regulated by GO:1903396; positively regulated by positive regulation of secondary cell septum biogenesis [GO:1903397] References: PMID:22891259